{
  "term_id": "GO:0032543",
  "gene": "UniProtKB:P82930",
  "term_label": "mitochondrial translation",
  "gene_name": "Small ribosomal subunit protein mS34",
  "gene_symbol": "MRPS34"
}